{
  "gene_name": "Katanin p60 ATPase-containing subunit A1",
  "gene": "UniProtKB:O75449",
  "gene_symbol": "KATNA1",
  "term_id": "GO:0051013",
  "term_label": "microtubule severing"
}